podocyte cell migration [GO:0090521] (biological process) Definition: The orderly movement of a podocyte from one site to another, often during the development of a multicellular organism or multicellular structure. A podocyte is a specialized kidney epithelial cell. Also known as: glomerular visceral epithelial cell migration References: PMID:21402783 Sources: GOC:pm Relationships: is a type of GO:0010631